establishment or maintenance of cytoskeleton polarity involved in mesendodermal cell migration [GO:0003372] (biological process) Definition: Any cellular process that results in the specification, formation or maintenance of polarized cytoskeletal structures that contribute to the cell polarity of a migrating mesendodermal cell. Sources: GOC:ascb_2009, GOC:dph, GOC:tb Relationships: is a type of establishment or maintenance of cytoskeleton polarity involved in gastrulation [GO:0003380]; is part of GO:0003369